{
  "term_id": "UNKNOWN:0003",
  "gene": "UniProtKB:Q14CZ0",
  "term_label": "Unknown cellular component",
  "gene_name": "HUWE1-associated protein modifying stress responses 1",
  "gene_symbol": "HAPSTR1"
}